{
  "gene": "UniProtKB:Q9Y320",
  "term_label": "brain development",
  "gene_symbol": "TMX2",
  "gene_name": "Thioredoxin-related transmembrane protein 2",
  "term_id": "GO:0007420"
}